cardiac muscle tissue morphogenesis [GO:0055008] (biological process) Definition: The process in which the anatomical structures of cardiac muscle tissue are generated and organized. Relationships: is a type of muscle tissue morphogenesis [GO:0060415]; is part of heart morphogenesis [GO:0003007]; is part of cardiac muscle tissue development [GO:0048738] Sources: GOC:devbiol Also known as: myocardium morphogenesis, heart muscle morphogenesis Subtypes: atrial cardiac muscle tissue morphogenesis [GO:0055009], GO:0055010